{
  "gene_symbol": "RBM28",
  "gene_name": "RNA-binding protein 28",
  "term_id": "UNKNOWN:0002",
  "gene": "UniProtKB:Q9NW13",
  "term_label": "Unknown biological process"
}